{
  "term_label": "cell surface receptor signaling pathway",
  "gene": "UniProtKB:O00463",
  "gene_symbol": "TRAF5",
  "gene_name": "TNF receptor-associated factor 5",
  "term_id": "GO:0007166"
}